cellular response to ecdysone [GO:0071390] (biological process) Relationships: is a type of response to ecdysone [GO:0035075]; is a type of cellular response to sterol [GO:0036315]; is a type of cellular response to alcohol [GO:0097306]; is a type of cellular response to ketone [GO:1901655] Definition: Any process that results in a change in state or activity of a cell (in terms of movement, secretion, enzyme production, gene expression, etc.) as a result of a ecdysone stimulus. Sources: GOC:mah